{
  "term_id": "GO:0005634",
  "gene": "UniProtKB:Q92731",
  "gene_name": "Estrogen receptor beta",
  "gene_symbol": "ESR2",
  "term_label": "nucleus"
}